{
  "gene": "UniProtKB:P09661",
  "gene_symbol": "SNRPA1",
  "term_label": "mRNA splicing, via spliceosome",
  "gene_name": "U2 small nuclear ribonucleoprotein A'",
  "term_id": "GO:0000398"
}